nucleotide-binding oligomerization domain containing 1 signaling pathway [GO:0070427] (biological process) References: PMID:17944960, PMID:18585455 Sources: GOC:add Relationships: is a type of nucleotide-binding domain, leucine rich repeat containing receptor signaling pathway [GO:0035872] Regulation: regulated by GO:0070428; negatively regulated by GO:0070429; positively regulated by positive regulation of nucleotide-binding oligomerization domain containing 1 signaling pathway [GO:0070430] Definition: The series of molecular signals initiated by the binding of a ligand (such as a bacterial peptidoglycan) to a cytoplasmic nucleotide-binding oligomerization domain containing 1 (NOD1) protein receptor, and ending with regulation of a downstream cellular process. Also known as: NOD1 signaling pathway, nucleotide-binding oligomerization domain containing 1 signalling pathway